{
  "term_id": "GO:0044322",
  "term_label": "endoplasmic reticulum quality control compartment",
  "gene_name": "F-box only protein 6",
  "gene": "UniProtKB:Q9NRD1",
  "gene_symbol": "FBXO6"
}